{
  "term_id": "GO:0006357",
  "gene": "UniProtKB:O95718",
  "gene_name": "Steroid hormone receptor ERR2",
  "term_label": "regulation of transcription by RNA polymerase II",
  "gene_symbol": "ESRRB"
}